{
  "term_id": "GO:0005886",
  "gene": "UniProtKB:P78369",
  "gene_symbol": "CLDN10",
  "term_label": "plasma membrane",
  "gene_name": "Claudin-10"
}